{
  "term_label": "phospholipid binding",
  "gene": "UniProtKB:Q9NZK7",
  "gene_symbol": "PLA2G2E",
  "gene_name": "Group IIE secretory phospholipase A2",
  "term_id": "GO:0005543"
}